{
  "term_label": "mitotic spindle organization",
  "gene_name": "Aurora kinase B",
  "gene": "UniProtKB:Q96GD4",
  "term_id": "GO:0007052",
  "gene_symbol": "AURKB"
}